{
  "gene": "UniProtKB:P78563",
  "gene_symbol": "ADARB1",
  "gene_name": "Double-stranded RNA-specific editase 1",
  "term_id": "GO:0005730",
  "term_label": "nucleolus"
}